cellular response to nickel ion [GO:0071289] (biological process) Definition: Any process that results in a change in state or activity of a cell (in terms of movement, secretion, enzyme production, gene expression, etc.) as a result of a nickel ion stimulus. Also known as: cellular response to nickel Relationships: is a type of response to nickel cation [GO:0010045]; is a type of GO:0071248 Sources: GOC:mah